{
  "gene_symbol": "NLK",
  "term_id": "GO:0005737",
  "gene": "UniProtKB:Q9UBE8",
  "term_label": "cytoplasm",
  "gene_name": "Serine_threonine-protein kinase NLK"
}